{
  "gene_symbol": "HCRT",
  "term_label": "positive regulation of transmission of nerve impulse",
  "gene_name": "Hypocretin neuropeptide precursor",
  "term_id": "GO:0051971",
  "gene": "UniProtKB:O43612"
}